{
  "gene": "UniProtKB:Q7L0Y3",
  "gene_name": "tRNA methyltransferase 10 homolog C",
  "term_id": "GO:0000049",
  "gene_symbol": "TRMT10C",
  "term_label": "tRNA binding"
}